{
  "gene_name": "Signal transducer and activator of transcription 6",
  "gene": "UniProtKB:P42226",
  "term_label": "growth hormone receptor signaling pathway via JAK-STAT",
  "gene_symbol": "STAT6",
  "term_id": "GO:0060397"
}